{
  "gene_symbol": "SMAP",
  "term_label": "Unknown cellular component",
  "gene": "UniProtKB:O00193",
  "term_id": "UNKNOWN:0003",
  "gene_name": "Small acidic protein"
}